{
  "term_label": "1-phosphatidylinositol-3-kinase activity",
  "term_id": "GO:0016303",
  "gene_symbol": "PIK3CD",
  "gene_name": "Phosphatidylinositol 4,5-bisphosphate 3-kinase catalytic subunit delta isoform",
  "gene": "UniProtKB:O00329"
}